{
  "gene_name": "Constitutive coactivator of PPAR-gamma-like protein 2",
  "gene": "UniProtKB:Q9NX05",
  "term_id": "UNKNOWN:0002",
  "gene_symbol": "FAM120C",
  "term_label": "Unknown biological process"
}